{
  "gene": "UniProtKB:O15347",
  "term_label": "Unknown molecular function",
  "gene_name": "High mobility group protein B3",
  "gene_symbol": "HMGB3",
  "term_id": "UNKNOWN:0001"
}